{
  "gene_name": "Omega-hydroxyceramide transacylase",
  "gene": "UniProtKB:Q8N8W4",
  "term_label": "triacylglycerol lipase activity",
  "gene_symbol": "PNPLA1",
  "term_id": "GO:0004806"
}